glomerular epithelial cell fate commitment [GO:0072314] (biological process) Definition: The process in which the developmental fate of a cell becomes restricted such that it will develop into a glomerular epithelial cell. Glomerular epithelial cells are specialized epithelial cells that form part of the glomerulus; there are two types, glomerular parietal epithelial cells and glomerular visceral epithelial cells. Sources: GOC:mtg_kidney_jan10 Subtypes: mesonephric glomerular epithelial cell fate commitment [GO:0061252], glomerular parietal epithelial cell fate commitment [GO:0072147], podocyte cell fate commitment [GO:0072149], metanephric glomerular epithelial cell fate commitment [GO:0072315] Relationships: is a type of GO:0002064; is part of glomerular epithelial cell differentiation [GO:0072311]